{
  "term_id": "UNKNOWN:0001",
  "gene_symbol": "Q8N8P6",
  "term_label": "Unknown molecular function",
  "gene": "UniProtKB:Q8N8P6",
  "gene_name": "Putative uncharacterized protein FLJ39060"
}